{
  "term_label": "intracellular signal transduction",
  "term_id": "GO:0035556",
  "gene_name": "STE20-like serine_threonine-protein kinase",
  "gene": "UniProtKB:Q9H2G2",
  "gene_symbol": "SLK"
}